{
  "term_label": "cytosol",
  "gene_name": "Microtubule-associated protein 1A",
  "gene_symbol": "MAP1A",
  "term_id": "GO:0005829",
  "gene": "UniProtKB:P78559"
}